{
  "gene_name": "Serine_threonine-protein kinase tousled-like 2",
  "gene": "UniProtKB:Q86UE8",
  "gene_symbol": "TLK2",
  "term_label": "nucleus",
  "term_id": "GO:0005634"
}